{
  "gene_symbol": "SLC25A11",
  "gene_name": "Mitochondrial 2-oxoglutarate_malate carrier protein",
  "term_label": "mitochondrial inner membrane",
  "gene": "UniProtKB:Q02978",
  "term_id": "GO:0005743"
}